{
  "gene_name": "Fc receptor-like protein 6",
  "gene_symbol": "FCRL6",
  "gene": "UniProtKB:Q6DN72",
  "term_id": "GO:0009897",
  "term_label": "external side of plasma membrane"
}